{
  "term_label": "mitotic metaphase chromosome alignment",
  "gene": "UniProtKB:Q6NXT2",
  "gene_name": "Histone H3.3C",
  "gene_symbol": "H3-5",
  "term_id": "GO:0007080"
}